{
  "gene_name": "Putative uncharacterized protein FLJ45035",
  "gene": "UniProtKB:Q6ZQT0",
  "term_label": "Unknown biological process",
  "term_id": "UNKNOWN:0002",
  "gene_symbol": "Q6ZQT0"
}